{
  "term_label": "Unknown biological process",
  "gene": "UniProtKB:E5RJM6",
  "gene_symbol": "ANKRD65",
  "term_id": "UNKNOWN:0002",
  "gene_name": "Ankyrin repeat domain-containing protein 65"
}